{
  "gene": "UniProtKB:P06681",
  "gene_symbol": "C2",
  "gene_name": "Complement C2",
  "term_label": "response to bacterium",
  "term_id": "GO:0009617"
}